mitochondrial alanyl-tRNA aminoacylation [GO:0070143] (biological process) Sources: GOC:mah, GOC:mcc Relationships: is a type of alanyl-tRNA aminoacylation [GO:0006419]; is a type of tRNA aminoacylation for mitochondrial protein translation [GO:0070127] Definition: The process of coupling alanine to alanyl-tRNA in a mitochondrion, catalyzed by alanyl-tRNA synthetase. In tRNA aminoacylation, the amino acid is first activated by linkage to AMP and then transferred to either the 2'- or the 3'-hydroxyl group of the 3'-adenosine residue of the tRNA.